{
  "gene": "UniProtKB:P36508",
  "term_label": "DNA-binding transcription factor activity, RNA polymerase II-specific",
  "term_id": "GO:0000981",
  "gene_name": "Zinc finger protein 76",
  "gene_symbol": "ZNF76"
}